{
  "gene_name": "Microfibrillar-associated protein 1",
  "term_label": "mRNA splicing, via spliceosome",
  "gene": "UniProtKB:P55081",
  "term_id": "GO:0000398",
  "gene_symbol": "MFAP1"
}